{
  "gene_name": "Doublesex- and mab-3-related transcription factor A1",
  "gene": "UniProtKB:Q5VZB9",
  "term_label": "DNA-binding transcription factor activity, RNA polymerase II-specific",
  "term_id": "GO:0000981",
  "gene_symbol": "DMRTA1"
}